{
  "gene_symbol": "LPGAT1",
  "term_label": "acyltransferase activity",
  "gene_name": "Acyl-CoA:lysophosphatidylglycerol acyltransferase 1",
  "term_id": "GO:0016746",
  "gene": "UniProtKB:Q92604"
}